{
  "gene": "UniProtKB:O00469",
  "term_label": "endoplasmic reticulum",
  "term_id": "GO:0005783",
  "gene_symbol": "PLOD2",
  "gene_name": "Procollagen-lysine,2-oxoglutarate 5-dioxygenase 2"
}